{
  "gene": "UniProtKB:Q9Y3A0",
  "term_id": "GO:0120539",
  "gene_name": "Ubiquinone biosynthesis protein COQ4 homolog, mitochondrial",
  "term_label": "4-hydroxy-3-methoxy-5-polyprenylbenzoate decarboxylase activity",
  "gene_symbol": "COQ4"
}